peptidyl-L-amino acid racemization [GO:0018085] (biological process) Definition: The process of conversion of a L-amino acid into its enantiomer, the corresponding D-amino acid. Subtypes: peptidyl-D-alanine racemization [GO:0019122] Sources: GOC:ma Relationships: is a type of peptidyl-amino acid modification [GO:0018193]; is a type of chiral amino acid racemization [GO:0018366]